tracheoesophageal septum formation [GO:1905327] (biological process) Relationships: is a type of anatomical structure formation involved in morphogenesis [GO:0048646] References: PMID:9731532 Sources: GOC:TermGenie, GO_REF:0000081 Definition: The process that gives rise to the tracheoesophageal septum. This process pertains to the initial formation of a structure from unspecified parts. Also known as: esophagotracheal septum formation, tracheoesophageal ridges formation